gamma-tubulin complex localization to nuclear side of mitotic spindle pole body [GO:0110120] (biological process) References: PMID:19942852 Sources: GOC:vw Definition: Any process in which a gamma-tubulin complex is transported to, or maintained in, a specific location at the nuclear side of the mitotic spindle pole body. Relationships: is a type of gamma-tubulin complex localization to mitotic spindle pole body [GO:1990735]